{
  "term_label": "Unknown biological process",
  "term_id": "UNKNOWN:0002",
  "gene_name": "Biogenesis of lysosome-related organelles complex 1 subunit 3",
  "gene": "UniProtKB:Q6QNY0",
  "gene_symbol": "BLOC1S3"
}